mesodermal cell differentiation [GO:0048333] (biological process) Regulation: regulated by regulation of mesodermal cell differentiation [GO:1905770]; RO_0002212 by negative regulation of mesodermal cell differentiation [GO:1905771]; positively regulated by positive regulation of mesodermal cell differentiation [GO:1905772] Sources: GOC:dgh Definition: The process in which a relatively unspecialized cell acquires the specialized features of a mesoderm cell. Also known as: mesoderm cell differentiation Subtypes: GO:0048321, paraxial mesodermal cell differentiation [GO:0048342], lateral mesodermal cell differentiation [GO:0048371], intermediate mesodermal cell differentiation [GO:0048392], GO:0060217 Relationships: is a type of GO:0030154; is part of mesoderm formation [GO:0001707]